protein-containing complex [GO:0032991] (cellular component) Also known as: macromolecular complex, macromolecule complex, protein containing complex, protein complex, protein-protein complex Relationships: is a type of cellular_component [GO:0005575] Sources: GOC:dos, GOC:mah Note: A protein complex in this context is meant as a stable set of interacting proteins which can be co-purified by an acceptable method, and where the complex has been shown to exist as an isolated, functional unit in vivo. Acceptable experimental methods include stringent protein purification followed by detection of protein interaction. The following methods should be considered non-acceptable: simple immunoprecipitation, pull-down experiments from cell extracts without further purification, colocalization and 2-hybrid screening. Interactions that should not be captured as protein complexes include: 1) enzyme/substrate, receptor/ligand or any similar transient interactions, unless these are a critical part of the complex assembly or are required e.g. for the receptor to be functional; 2) proteins associated in a pull-down/co-immunoprecipitation assay with no functional link or any evidence that this is a defined biological entity rather than a loose-affinity complex; 3) any complex where the only evidence is based on genetic interaction data; 4) partial complexes, where some subunits (e.g. transmembrane ones) cannot be expressed as recombinant proteins and are excluded from experiments (in this case, independent evidence is necessary to find out the composition of the full complex, if known). Interactions that may be captured as protein complexes include: 1) enzyme/substrate or receptor/ligand if the complex can only assemble and become functional in the presence of both classes of subunits; 2) complexes where one of the members has not been shown to be physically linked to the other(s), but is a homologue of, and has the same functionality as, a protein that has been experimentally demonstrated to form a complex with the other member(s); 3) complexes whose existence is accepted based on localization and pharmacological studies, but for which experimental evidence is not yet available for the complex as a whole. Definition: A stable assembly of two or more macromolecules, i.e. proteins, nucleic acids, carbohydrates or lipids, in which at least one component is a protein and the constituent parts function together. Subtypes: polarisome [GO:0000133], HIR complex [GO:0000417], condensin complex [GO:0000796], GO:0000808, gamma-tubulin complex [GO:0000930], inner kinetochore [GO:0000939], outer kinetochore [GO:0000940], Prp19 complex [GO:0000974], GO:0001114, radial spoke [GO:0001534], radial spoke head [GO:0001535], GO:0001536, polkadots [GO:0002096], polycystin complex [GO:0002133], stereocilia ankle link complex [GO:0002142], VRK3/VHR/ERK complex [GO:0002167], MAML1-RBP-Jkappa- ICN1 complex [GO:0002193], GO:0002199, MECO complex [GO:0002929], GO:0005577, collagen trimer [GO:0005581], complement component C1 complex [GO:0005602], larval serum protein complex [GO:0005616], DNA replication factor C complex [GO:0005663], transcription regulator complex [GO:0005667], steroid hormone aporeceptor complex [GO:0005831], GO:0005833, proteasome regulatory particle [GO:0005838], eukaryotic translation initiation factor 2 complex [GO:0005850], GO:0005852, eukaryotic translation elongation factor 1 complex [GO:0005853], nascent polypeptide-associated complex [GO:0005854], troponin complex [GO:0005861], muscle thin filament tropomyosin [GO:0005862], microtubule associated complex [GO:0005875], Arp2/3 protein complex [GO:0005885], axonemal nexin link [GO:0005931], GO:0008091, cohesin complex [GO:0008278], F-actin capping protein complex [GO:0008290], GO:0008537, GO:0008540, proteasome regulatory particle, lid subcomplex [GO:0008541], alkyl hydroperoxide reductase complex [GO:0009321], GO:0009390, GO:0015627, prefoldin complex [GO:0016272], myosin complex [GO:0016459], GO:0017102, translation release factor complex [GO:0018444], GO:0019035, viral transcriptional complex [GO:0019036], GO:0019773, proteasome core complex, beta-subunit complex [GO:0019774], GO:0019814, proteasome-activating nucleotidase complex [GO:0022623], GO:0022624, light-harvesting complex [GO:0030076], B875 antenna complex [GO:0030080], B800-820 antenna complex [GO:0030081], B800-850 antenna complex [GO:0030082], GO:0030256, GO:0030257, junctional membrane complex [GO:0030314], intraciliary transport particle [GO:0030990], intraciliary transport particle A [GO:0030991], intraciliary transport particle B [GO:0030992], axonemal heterotrimeric kinesin-II complex [GO:0030993], nucleocytoplasmic transport complex [GO:0031074], septin complex [GO:0031105], GO:0031209, Ndc80 complex [GO:0031262], Rad17 RFC-like complex [GO:0031389], bursicon neuropeptide hormone complex [GO:0031395], Mis6-Sim4 complex [GO:0031511], GO:0031521, G-protein beta/gamma-subunit complex [GO:0031680], haptoglobin-hemoglobin complex [GO:0031838], filamentous actin [GO:0031941], mismatch repair complex [GO:0032300], angiogenin-PRI complex [GO:0032311], NHE3/E3KARP/ACTN4 complex [GO:0032766], GO:0032777, protein-carbohydrate complex [GO:0032992], protein-DNA complex [GO:0032993], protein-lipid complex [GO:0032994], DNA recombinase mediator complex [GO:0033061], type VI protein secretion system complex [GO:0033104], GO:0033186, Lsd1/2 complex [GO:0033193], monopolin complex [GO:0033551], TSC1-TSC2 complex [GO:0033596], exomer complex [GO:0034044], Cvt complex [GO:0034270], BBSome [GO:0034464], Par3-APC-KIF3A complex [GO:0034748], Scrib-APC complex [GO:0034749], GO:0034750, Sid2-Mob1 complex [GO:0034973], RasGAP-Fyn-Lyn-Yes complex [GO:0034996], Nrd1 complex [GO:0035649], NOS2-CD74 complex [GO:0035693], Seh1-associated complex [GO:0035859], MKS complex [GO:0036038], tubulobulbar complex [GO:0036284], eisosome filament [GO:0036286], Kibra-Ex-Mer complex [GO:0036375], TCR signalosome [GO:0036398], ESCRT complex [GO:0036452], GO:0036454, UFD1-NPL4 complex [GO:0036501], GO:0038045, IKKalpha-IKKalpha complex [GO:0038059], TBK1-IKKE-DDX3 complex [GO:0039658], MCM complex [GO:0042555], GO:0043235, laminin complex [GO:0043256], RAVE complex [GO:0043291], apoptosome [GO:0043293], GO:0043493, inhibin complex [GO:0043511], interleukin-12 complex [GO:0043514], type IV secretion system complex [GO:0043684], RecFOR complex [GO:0043850], GO:0044697, GO:0044777, GO:0044816, GO:0045251, GO:0045298, viral portal complex [GO:0046798], viral scaffold [GO:0046806], GO:0048180, Ski complex [GO:0055087], GO:0061574, pituitary gonadotropin complex [GO:0061696], GATOR2 complex [GO:0061700], canonical inflammasome complex [GO:0061702], pyroptosome complex [GO:0061703], TOC-TIC supercomplex I [GO:0061927], NVT complex [GO:0061957], lymphotoxin complex [GO:0062048], protein phosphatase inhibitor complex [GO:0062049], histone mRNA stem-loop binding complex [GO:0062073], GO:0062092, complement component C1q complex [GO:0062167], GO:0070288, G-protein beta/gamma-Raf-1 complex [GO:0070422], G-protein beta/gamma-Btk complex [GO:0070441], GO:0070695, GO:0070743, interleukin-27 complex [GO:0070744], interleukin-35 complex [GO:0070745], paraferritin complex [GO:0070826], CUGBP1-eIF2 complex [GO:0071075], GO:0071141, WASH complex [GO:0071203], Myo2p-Vac17p-Vac8p transport complex [GO:0071563], MMXD complex [GO:0071817], ER membrane insertion complex [GO:0072379], FAR/SIN/STRIPAK complex [GO:0090443], GO:0090665, TRAF2-GSTP1 complex [GO:0097057], GO:0097058, CNTFR-CLCF1 complex [GO:0097059], interferon regulatory factor complex [GO:0097071], GO:0097078, Bcl-2 family protein complex [GO:0097136], GO:0097196, GO:0097255, TAM protein secretion complex [GO:0097347], MCM core complex [GO:0097373], GAIT complex [GO:0097452], H-NS-Hha complex [GO:0097495], Y-shaped link [GO:0097537], viral terminase, small subunit [GO:0097710], type V protein secretion system complex [GO:0098046], methyl accepting chemotaxis protein complex [GO:0098561], protein complex involved in cell adhesion [GO:0098636], hemidesmosome associated protein complex [GO:0098733], RNA decapping complex [GO:0098745], membrane protein complex [GO:0098796], mitochondrial protein-containing complex [GO:0098798], respiratory chain complex [GO:0098803], trans-synaptic protein complex [GO:0098820], GO:0099023, transforming growth factor beta complex [GO:0099126], GO:0106002, amyloid-beta complex [GO:0106003], EDS1 disease-resistance complex [GO:0106093], Nicalin-NOMO complex [GO:0106249], GO:0106333, TTT Hsp90 cochaperone complex [GO:0110078], Aim21-Tda2 complex [GO:0110131], reelin complex [GO:0110157], procentriole replication complex [GO:0120099], Sm-like protein family complex [GO:0120114], GO:0120124, MIH complex [GO:0120155], Cdc24p-Far1p-Gbetagamma complex [GO:0120171], GO:0120216, GO:0120228, radial spoke base [GO:0120339], radial spoke neck [GO:0120343], KICSTOR complex [GO:0140007], SLAC complex [GO:0140224], DNA topoisomerase III-beta-TDRD3 complex [GO:0140225], counting factor complex [GO:0140451], nuclear protein-containing complex [GO:0140513], endoplasmic reticulum protein-containing complex [GO:0140534], intracellular protein-containing complex [GO:0140535], iRhom2/ADAM17 sheddase complex [GO:0140910], GO:0150005, glideosome [GO:0160055], SIN/MEN signaling complex [GO:0160065], non-canonical inflammasome complex [GO:0160074], hemozoin formation complex [GO:0160092], FERRY complex [GO:0160271], sodium-translocating NADH:quinone reductase complex [GO:0160292], SKA complex [GO:0170027], CROP complex [GO:0170071], Knl1/Spc105 complex [GO:0180019], RQC-trigger complex [GO:0180022], Mrh5C translation activator complex [GO:0180049], GO:1902494, metallochaperone complex [GO:1902695], translation repressor complex [GO:1903502], ATPase inhibitor complex [GO:1903503], peptidase inhibitor complex [GO:1904090], Ras guanyl-nucleotide exchange factor complex [GO:1905742], RPAP3/R2TP/prefoldin-like complex [GO:1990062], Dxr protein complex [GO:1990065], replication inhibiting complex [GO:1990078], GO:1990100, DNA bending complex [GO:1990104], RQC complex [GO:1990112], DiaA complex [GO:1990125], GATOR1 complex [GO:1990130], SsuD-SsuE complex [GO:1990200], iron-sulfur cluster assembly complex [GO:1990229], nucleotide-excision repair, DNA damage recognition complex [GO:1990249], Syp1 complex [GO:1990252], bub1-bub3 complex [GO:1990298], GO:1990315, thrombospondin complex [GO:1990341], GO:1990346, GO:1990351, 3M complex [GO:1990393], RZZ complex [GO:1990423], lateral cortical node [GO:1990463], raps-insc complex [GO:1990499], PYM-mago-Y14 complex [GO:1990509], Ste12p-Dig1p-Dig2p complex [GO:1990526], Tec1p-Ste12p-Dig1p complex [GO:1990527], Rvs161p-Rvs167p complex [GO:1990528], GO:1990533, extracellular exosome complex [GO:1990563], divisome complex [GO:1990586], AIP1-IRE1 complex [GO:1990597], Kelch-containing formin regulatory complex [GO:1990615], GO:1990630, calprotectin complex [GO:1990660], S100A8 complex [GO:1990661], GO:1990665, PCSK9-LDLR complex [GO:1990666], PCSK9-AnxA2 complex [GO:1990667], GO:1990682, GO:1990684, GO:1990696, MAD1 complex [GO:1990706], tubulin folding cofactor complex [GO:1990727], mitotic spindle assembly checkpoint MAD1-MAD2 complex [GO:1990728], VCP-NSFL1C complex [GO:1990730], titin-telethonin complex [GO:1990733], EARP complex [GO:1990745], GLI-SUFU complex [GO:1990788], MWP complex [GO:1990811], Vma12-Vma22 assembly complex [GO:1990871], ribonucleoprotein complex [GO:1990904], GO:1990909, PET complex [GO:1990923], GO:1990957, GO:1990964